{
  "gene_symbol": "RDH11",
  "term_label": "Unknown biological process",
  "term_id": "UNKNOWN:0002",
  "gene": "UniProtKB:Q8TC12",
  "gene_name": "Retinol dehydrogenase 11"
}